{
  "gene_name": "Olfactory receptor 10H4",
  "term_label": "olfactory receptor activity",
  "gene_symbol": "OR10H4",
  "term_id": "GO:0004984",
  "gene": "UniProtKB:Q8NGA5"
}